{
  "gene_name": "Immunoglobulin heavy variable 3-30-3",
  "term_id": "GO:0016064",
  "term_label": "immunoglobulin mediated immune response",
  "gene_symbol": "IGHV3-30-3",
  "gene": "UniProtKB:P0DP02"
}